response to pain [GO:0048265] (biological process) Also known as: physiological response to pain References: PMID:10203867, PMID:12723742, PMID:12843304 Sources: GOC:jid, Wikipedia:Pain Relationships: is a type of multicellular organismal response to stress [GO:0033555] Definition: Any process that results in a change in state or activity of a cell or an organism (in terms of movement, secretion, enzyme production, gene expression, etc.) as a result of a pain stimulus. Pain stimuli cause activation of nociceptors, peripheral receptors for pain, include receptors which are sensitive to painful mechanical stimuli, extreme heat or cold, and chemical stimuli.